{
  "term_id": "GO:0005948",
  "gene": "UniProtKB:A1L0T0",
  "gene_name": "2-hydroxyacyl-CoA lyase 2",
  "gene_symbol": "ILVBL",
  "term_label": "acetolactate synthase complex"
}